{
  "gene_name": "Switch-associated protein 70",
  "term_id": "UNKNOWN:0002",
  "term_label": "Unknown biological process",
  "gene": "UniProtKB:Q9UH65",
  "gene_symbol": "SWAP70"
}